release of sequestered calcium ion into cytosol [GO:0051209] (biological process) Definition: The process in which calcium ions sequestered in the endoplasmic reticulum, Golgi apparatus or mitochondria are released into the cytosolic compartment. Regulation: regulated by regulation of release of sequestered calcium ion into cytosol [GO:0051279]; RO_0002212 by negative regulation of release of sequestered calcium ion into cytosol [GO:0051280]; positively regulated by positive regulation of release of sequestered calcium ion into cytosol [GO:0051281] References: PMID:1814929 Sources: GOC:dph, GOC:hjd, GOC:mtg_lung Also known as: calcium ion (Ca2+) mobilization, calcium mobilization, cytoplasmic release of sequestered calcium ion (Ca2+), cytoplasmic release of stored calcium ion (Ca2+), release of sequestered calcium ion (Ca2+), release of sequestered calcium ion into cytoplasm, release of stored calcium ion (Ca2+), release of stored calcium ion (Ca2+) into cytoplasm, cytosolic release of sequestered calcium ion (Ca2+), cytosolic release of stored calcium ion (Ca2+), release of stored calcium ion (Ca2+) into cytosol Relationships: is_a negative regulation of sequestering of calcium ion [GO:0051283]; is a type of calcium ion transmembrane import into cytosol [GO:0097553] Subtypes: release of sequestered calcium ion into cytosol by Golgi [GO:0061454], GO:0099093, GO:0099585, GO:0099586, release of sequestered calcium ion into cytosol by endoplasmic reticulum [GO:1903514]